{
  "gene_name": "UL-16 binding protein 5",
  "gene_symbol": "RAET1G",
  "gene": "UniProtKB:Q6H3X3",
  "term_label": "natural killer cell mediated cytotoxicity",
  "term_id": "GO:0042267"
}